{
  "gene_symbol": "C8orf88",
  "term_id": "UNKNOWN:0003",
  "gene_name": "Uncharacterized protein C8orf88",
  "gene": "UniProtKB:P0DMB2",
  "term_label": "Unknown cellular component"
}